{
  "gene_name": "5-hydroxytryptamine receptor 3B",
  "term_label": "chemical synaptic transmission",
  "term_id": "GO:0007268",
  "gene_symbol": "HTR3B",
  "gene": "UniProtKB:O95264"
}